cerebellar Purkinje cell layer maturation [GO:0021691] (biological process) Relationships: is a type of GO:0071695; is part of cerebellar Purkinje cell layer development [GO:0021680]; is part of cerebellar cortex maturation [GO:0021699] Definition: A developmental process, independent of morphogenetic (shape) change, that is required for the cerebellar Purkinje cell layer to attain its fully functional state. The Purkinje cell layer lies just underneath the molecular layer of the cerebellar cortex. It contains the neuronal cell bodies of the Purkinje cells that are arranged side by side in a single layer. Candelabrum interneurons are vertically oriented between the Purkinje cells. Purkinje neurons are inhibitory and provide the output of the cerebellar cortex through axons that project into the white matter. Extensive dendritic trees from the Purkinje cells extend upward in a single plane into the molecular layer where they synapse with parallel fibers of granule cells. Sources: GOC:cls, GOC:dgh, GOC:dph, GOC:jid, GO_REF:0000021